{
  "gene_name": "Junction plakoglobin",
  "gene": "UniProtKB:P14923",
  "gene_symbol": "JUP",
  "term_label": "catenin complex",
  "term_id": "GO:0016342"
}